mammillary body development [GO:0021767] (biological process) Relationships: is a type of anatomical structure development [GO:0048856]; BFO_0000050 diencephalon development [GO:0021536]; is part of limbic system development [GO:0021761] Sources: GOC:cls, GOC:dgh, GOC:dph, GOC:jid, GO_REF:0000021 Definition: The progression of the mammillary body over time from its initial formation until its mature state. The mammillary body is a protrusion at the posterior end of the hypothalamus that contains hypothalamic nuclei.